{
  "term_id": "GO:0000978",
  "gene_symbol": "SOX13",
  "gene": "UniProtKB:Q9UN79",
  "term_label": "RNA polymerase II cis-regulatory region sequence-specific DNA binding",
  "gene_name": "Transcription factor SOX-13"
}